{
  "gene_name": "ADP-ribosylation factor-like protein 4D",
  "gene_symbol": "ARL4D",
  "gene": "UniProtKB:P49703",
  "term_label": "GTP binding",
  "term_id": "GO:0005525"
}